{
  "term_label": "Unknown molecular function",
  "gene": "UniProtKB:A2NJV5",
  "gene_name": "Immunoglobulin kappa variable 2-29",
  "term_id": "UNKNOWN:0001",
  "gene_symbol": "IGKV2-29"
}